{
  "gene_symbol": "HSPD1",
  "gene_name": "60 kDa heat shock protein, mitochondrial",
  "gene": "UniProtKB:P10809",
  "term_label": "positive regulation of interferon-alpha production",
  "term_id": "GO:0032727"
}